protein processing in phagocytic vesicle [GO:1900756] (biological process) Sources: GOC:TermGenie, GOC:rjd Definition: Protein processing that takes place in the phagosome. Most protein processing in the phagosome represents protein degradation. Relationships: is a type of protein processing [GO:0016485]; occurs in phagocytic vesicle [GO:0045335] Also known as: protein maturation by peptide bond cleavage in phagocytic vesicle, protein maturation by peptide bond cleavage in phagosome, protein maturation by peptide bond hydrolysis in phagocytic vesicle, protein maturation by peptide bond hydrolysis in phagosome, protein processing in phagosome, peptidolysis during protein maturation in phagocytic vesicle, peptidolysis during protein maturation in phagosome, protein maturation by proteolysis in phagocytic vesicle, protein maturation by proteolysis in phagosome Regulation: regulated by regulation of protein processing in phagocytic vesicle [GO:1903921]; negatively regulated by negative regulation of protein processing in phagocytic vesicle [GO:1903922]; RO_0002213 by positive regulation of protein processing in phagocytic vesicle [GO:1903923]